{
  "gene_symbol": "FAM90A7",
  "term_label": "Unknown cellular component",
  "gene": "UniProtKB:A6NKC0",
  "gene_name": "Putative protein FAM90A7",
  "term_id": "UNKNOWN:0003"
}